{
  "gene_symbol": "ZNF767P",
  "gene": "UniProtKB:Q75MW2",
  "term_id": "UNKNOWN:0002",
  "term_label": "Unknown biological process",
  "gene_name": "Protein ZNF767"
}